3-hydroxypropionate dehydrogenase (NAD+) activity [GO:0047565] (molecular function) Definition: Catalysis of the reaction: 3-hydroxypropanoate + NAD+ = 3-oxopropanoate + H+ + NADH. Sources: EC:1.1.1.59, RHEA:13357 Also known as: 3-hydroxypropanoate:NAD+ oxidoreductase activity Relationships: is a type of oxidoreductase activity, acting on the CH-OH group of donors, NAD or NADP as acceptor [GO:0016616]